{
  "term_id": "GO:0006357",
  "gene": "UniProtKB:Q96JF6",
  "gene_symbol": "ZNF594",
  "gene_name": "Zinc finger protein 594",
  "term_label": "regulation of transcription by RNA polymerase II"
}